{
  "term_label": "mitochondrial respiratory chain complex IV assembly",
  "term_id": "GO:0033617",
  "gene_symbol": "COA1",
  "gene": "UniProtKB:Q9GZY4",
  "gene_name": "Cytochrome c oxidase assembly factor 1 homolog"
}